{
  "gene": "UniProtKB:Q96HZ4",
  "gene_name": "Transcription cofactor HES-6",
  "gene_symbol": "HES6",
  "term_label": "nucleus",
  "term_id": "GO:0005634"
}